LPPG:FO 2-phospho-L-lactate transferase activity [GO:0043743] (molecular function) Relationships: is_a phosphotransferase activity, alcohol group as acceptor [GO:0016773] References: PMID:11888293 Definition: Catalysis of the reaction: 7,8-didemethyl-8-hydroxy-5-deazariboflavin + lactyl-2-diphospho-5'-guanosine = coenzyme F420-0 + GMP.